{
  "term_label": "Unknown molecular function",
  "gene_symbol": "C4orf33",
  "gene": "UniProtKB:Q8N1A6",
  "gene_name": "UPF0462 protein C4orf33",
  "term_id": "UNKNOWN:0001"
}